{
  "gene_name": "Muscarinic acetylcholine receptor M2",
  "gene": "UniProtKB:P08172",
  "term_label": "dendrite",
  "term_id": "GO:0030425",
  "gene_symbol": "CHRM2"
}